{
  "gene_symbol": "BCL10",
  "gene": "UniProtKB:O95999",
  "gene_name": "B-cell lymphoma_leukemia 10",
  "term_id": "GO:0019209",
  "term_label": "kinase activator activity"
}